{
  "term_label": "Unknown molecular function",
  "term_id": "UNKNOWN:0001",
  "gene_symbol": "MAGEF1",
  "gene_name": "Melanoma-associated antigen F1",
  "gene": "UniProtKB:Q9HAY2"
}